gonadotrophin-releasing hormone neuronal migration to the hypothalamus [GO:0021828] (BP) References: PMID:12626695 Sources: GOC:cls, GOC:dgh, GOC:dph, GOC:jid, GO_REF:0000021 Also known as: gonadotropin-releasing hormone neuronal migration to the hypothalamus Relationships: is a type of neuron migration [GO:0001764]; is_a hypothalamic tangential migration using cell-axon interactions [GO:0021856]; is part of GO:0021888 Definition: The directional movement of a gonadotrophin-releasing hormone producing neuron from the nasal placode to the hypothalamus.